{
  "gene_name": "FERM domain-containing protein 4A",
  "gene_symbol": "FRMD4A",
  "term_label": "adherens junction",
  "gene": "UniProtKB:Q9P2Q2",
  "term_id": "GO:0005912"
}